{
  "term_id": "GO:0031783",
  "gene_symbol": "MRAP2",
  "gene_name": "Melanocortin-2 receptor accessory protein 2",
  "term_label": "type 5 melanocortin receptor binding",
  "gene": "UniProtKB:Q96G30"
}